negative regulation of calcium ion import across plasma membrane [GO:1905949] (biological process) References: PMID:17640527 Sources: GOC:TermGenie, GOC:bhm, GO_REF:0000058 Note: An example of this is PPP3CA in human (Q08209) in PMID:17640527 (inferred from direct assay). Definition: Any process that stops, prevents or reduces the frequency, rate or extent of calcium ion import across plasma membrane. Also known as: down regulation of calcium ion import across plasma membrane, down-regulation of calcium ion import across plasma membrane, downregulation of calcium ion import across plasma membrane, inhibition of calcium ion import across plasma membrane Relationships: is a type of GO:0090281; is a type of GO:1903170; is a type of regulation of calcium ion import across plasma membrane [GO:1905664]; RO_0002212 GO:0098703